{
  "gene": "UniProtKB:Q99704",
  "term_label": "Ras protein signal transduction",
  "term_id": "GO:0007265",
  "gene_name": "Docking protein 1",
  "gene_symbol": "DOK1"
}